{
  "term_label": "proteasome-mediated ubiquitin-dependent protein catabolic process",
  "gene_name": "PRAME family member 17",
  "term_id": "GO:0043161",
  "gene": "UniProtKB:Q5VTA0",
  "gene_symbol": "PRAMEF17"
}